regulation of taurine biosynthetic process [GO:0062089] (biological process) Subtypes: positive regulation of taurine biosynthetic process [GO:0062090] References: PMID:18648510, PMID:24911144 Sources: GOC:BHF Definition: Any process that modulates the rate, frequency or extent of taurine biosynthesis. Relationships: is_a regulation of biosynthetic process [GO:0009889]; is a type of GO:0042762; is a type of regulation of small molecule metabolic process [GO:0062012]; regulates taurine biosynthetic process [GO:0042412]